{
  "gene": "UniProtKB:Q96N38",
  "gene_name": "Zinc finger protein 714",
  "gene_symbol": "ZNF714",
  "term_label": "Unknown cellular component",
  "term_id": "UNKNOWN:0003"
}